{
  "gene_symbol": "YJU2B",
  "gene": "UniProtKB:P13994",
  "gene_name": "Probable splicing factor YJU2B",
  "term_id": "GO:0045292",
  "term_label": "mRNA cis splicing, via spliceosome"
}